{
  "term_id": "GO:0005802",
  "gene": "UniProtKB:Q96DS6",
  "gene_name": "Membrane-spanning 4-domains subfamily A member 6E",
  "gene_symbol": "MS4A6E",
  "term_label": "trans-Golgi network"
}